medulla oblongata morphogenesis [GO:0021579] (biological process) Relationships: is a type of anatomical structure morphogenesis [GO:0009653]; is part of medulla oblongata development [GO:0021550]; is part of hindbrain morphogenesis [GO:0021575] Sources: GOC:cls, GOC:dgh, GOC:dph, GOC:jid, GO_REF:0000021 Also known as: medulla morphogenesis, myelencephalon morphogenesis Definition: The process in which the anatomical structure of the medulla oblongata is generated and organized. The medulla oblongata lies directly above the spinal cord and controls vital autonomic functions such as digestion, breathing and the control of heart rate.